{
  "term_id": "GO:0051087",
  "term_label": "protein-folding chaperone binding",
  "gene": "UniProtKB:O15212",
  "gene_name": "Prefoldin subunit 6",
  "gene_symbol": "PFDN6"
}